{
  "gene": "UniProtKB:Q9GZV7",
  "term_id": "GO:0007417",
  "gene_symbol": "HAPLN2",
  "gene_name": "Hyaluronan and proteoglycan link protein 2",
  "term_label": "central nervous system development"
}